{
  "term_label": "RNA polymerase II cis-regulatory region sequence-specific DNA binding",
  "gene": "UniProtKB:Q86UE3",
  "gene_name": "Zinc finger protein 546",
  "term_id": "GO:0000978",
  "gene_symbol": "ZNF546"
}